{
  "gene_name": "Protein S100-B",
  "term_id": "GO:0005615",
  "term_label": "extracellular space",
  "gene": "UniProtKB:P04271",
  "gene_symbol": "S100B"
}